{
  "gene_symbol": "HLA-DQB2",
  "gene": "UniProtKB:P05538",
  "gene_name": "HLA class II histocompatibility antigen, DQ beta 2 chain",
  "term_id": "GO:0031902",
  "term_label": "late endosome membrane"
}